positive regulation of austinol biosynthetic process [GO:1900642] (biological process) Definition: Any process that activates or increases the frequency, rate or extent of austinol biosynthetic process. Sources: GOC:TermGenie, GOC:di Also known as: activation of austinol anabolism, activation of austinol biosynthesis, activation of austinol formation, activation of austinol synthesis, positive regulation of austinol anabolism, positive regulation of austinol biosynthesis, positive regulation of austinol formation, positive regulation of austinol synthesis, up regulation of austinol anabolism, up regulation of austinol biosynthesis, up regulation of austinol biosynthetic process, up regulation of austinol formation, up regulation of austinol synthesis, up-regulation of austinol anabolism, up-regulation of austinol biosynthesis, up-regulation of austinol biosynthetic process, up-regulation of austinol formation, up-regulation of austinol synthesis, upregulation of austinol anabolism, upregulation of austinol biosynthesis, upregulation of austinol biosynthetic process, upregulation of austinol formation, upregulation of austinol synthesis, activation of austinol biosynthetic process Relationships: is a type of positive regulation of biosynthetic process [GO:0009891]; is a type of GO:1900640; positively regulates GO:1900560